{
  "term_label": "transcription corepressor activity",
  "gene_name": "Nuclear receptor corepressor 2",
  "gene": "UniProtKB:Q9Y618",
  "gene_symbol": "NCOR2",
  "term_id": "GO:0003714"
}